{
  "term_id": "UNKNOWN:0001",
  "gene_symbol": "PCARE",
  "term_label": "Unknown molecular function",
  "gene": "UniProtKB:A6NGG8",
  "gene_name": "Photoreceptor cilium actin regulator"
}